{
  "term_id": "GO:0007169",
  "gene_name": "Protein-tyrosine kinase 6",
  "term_label": "cell surface receptor protein tyrosine kinase signaling pathway",
  "gene_symbol": "PTK6",
  "gene": "UniProtKB:Q13882"
}